fibronectin fibril organization [GO:1905590] (biological process) References: PMID:20690820 Sources: GOC:TermGenie, GOC:dph Relationships: is a type of supramolecular fiber organization [GO:0097435] Definition: A process that is carried out at the cellular level which results in the assembly, arrangement of constituent parts, or disassembly of a fibronectin fibril.